protein secretion by the type I secretion system [GO:0030253] (biological process) Also known as: protein secretion by the TOSS, protein secretion by the type I protein secretion system, type I protein secretion system Definition: The process in which proteins are secreted into the extracellular milieu via the type I secretion system; secretion occurs in a continuous process without the distinct presence of periplasmic intermediates and does not involve proteolytic processing of secreted proteins. Relationships: is a type of protein secretion [GO:0009306]; is a type of protein transmembrane transport [GO:0071806] Note: Note that this term represents an activity and not a cellular structure. Consider also annotating to the cellular component term 'type I protein secretion system complex ; GO:0030256'. Sources: GOC:pamgo_curators